{
  "term_label": "Unknown molecular function",
  "gene_name": "Keratin-associated protein 15-1",
  "gene": "UniProtKB:Q3LI76",
  "gene_symbol": "KRTAP15-1",
  "term_id": "UNKNOWN:0001"
}